positive regulation of Schwann cell chemotaxis [GO:1904268] (biological process) Relationships: is a type of positive regulation of chemotaxis [GO:0050921]; is a type of positive regulation of Schwann cell migration [GO:1900149]; is a type of regulation of Schwann cell chemotaxis [GO:1904266]; positively regulates Schwann cell chemotaxis [GO:1990751] Definition: Any process that activates or increases the frequency, rate or extent of Schwann cell chemotaxis. References: PMID:16203995 Sources: GOC:TermGenie, GO_REF:0000058 Also known as: up regulation of Schwann cell chemotaxis, up-regulation of Schwann cell chemotaxis, upregulation of Schwann cell chemotaxis, activation of Schwann cell chemotaxis